{
  "gene_name": "Serine_arginine repetitive matrix protein 4",
  "term_label": "nucleus",
  "gene_symbol": "SRRM4",
  "term_id": "GO:0005634",
  "gene": "UniProtKB:A7MD48"
}